{
  "gene_symbol": "AP3B1",
  "term_label": "Unknown cellular component",
  "gene_name": "AP-3 complex subunit beta-1",
  "gene": "UniProtKB:O00203",
  "term_id": "UNKNOWN:0003"
}